pulmonary blood vessel remodeling [GO:0101010] (biological process) Also known as: pulmonary blood vessel remodelling Sources: GOC:mec Regulation: regulated by regulation of pulmonary blood vessel remodeling [GO:1905109]; negatively regulated by GO:1905110; positively regulated by positive regulation of pulmonary blood vessel remodeling [GO:1905111] Relationships: is a type of blood vessel remodeling [GO:0001974] Definition: The reorganization or renovation of existing pulmonary blood vessels.